{
  "gene": "UniProtKB:Q9HCS7",
  "term_id": "GO:0000349",
  "gene_symbol": "XAB2",
  "gene_name": "Pre-mRNA-splicing factor SYF1",
  "term_label": "generation of catalytic spliceosome for first transesterification step"
}